{
  "gene_name": "Golgin subfamily A member 8R",
  "gene": "UniProtKB:I6L899",
  "gene_symbol": "GOLGA8R",
  "term_label": "Golgi organization",
  "term_id": "GO:0007030"
}